regulation of neurotransmitter uptake [GO:0051580] (biological process) Sources: GOC:ai Also known as: regulation of neurotransmitter import, regulation of neurotransmitter reuptake Relationships: is a type of GO:0051588; regulates neurotransmitter uptake [GO:0001504] Definition: Any process that modulates the frequency, rate or extent of the directed movement of a neurotransmitter into a neuron or glial cell. Subtypes: negative regulation of neurotransmitter uptake [GO:0051581], GO:0051582, regulation of serotonin uptake [GO:0051611], regulation of histamine uptake [GO:0051616], regulation of catecholamine uptake involved in synaptic transmission [GO:0051940], regulation of amino acid uptake involved in synaptic transmission [GO:0051941]